phloem glucosinolate loading [GO:0090449] (biological process) References: PMID:22864417 Definition: The process of loading glucosinolates into the sieve tube or companion cell of the phloem for long distance transport from source to sink. Relationships: is_a phloem loading [GO:0110126]; is a type of glucosinolate transport [GO:1901349]